purine nucleoside biosynthetic process [GO:0042451] (biological process) Subtypes: purine deoxyribonucleoside biosynthetic process [GO:0046123], GO:0046129 Definition: The chemical reactions and pathways resulting in the formation of any purine nucleoside, one of a family of organic molecules consisting of a purine base covalently bonded to a sugar ribose (a ribonucleoside) or deoxyribose (a deoxyribonucleoside). Also known as: purine nucleoside anabolism, purine nucleoside biosynthesis, purine nucleoside formation, purine nucleoside synthesis Sources: GOC:go_curators Relationships: is a type of nucleoside biosynthetic process [GO:0009163]; is a type of purine nucleoside metabolic process [GO:0042278]; is a type of purine-containing compound biosynthetic process [GO:0072522]